{
  "term_label": "transmembrane signaling receptor activity",
  "gene_symbol": "KIR2DP1",
  "gene_name": "Killer cell immunoglobulin-like receptor, two Ig domains pseudogene 1",
  "gene": "UniProtKB:A0A0G2JNF4",
  "term_id": "GO:0004888"
}